{
  "gene": "UniProtKB:Q92851",
  "term_label": "cytoplasm",
  "term_id": "GO:0005737",
  "gene_symbol": "CASP10",
  "gene_name": "Caspase-10"
}